{
  "term_label": "mRNA regulatory element binding translation repressor activity",
  "term_id": "GO:0000900",
  "gene_symbol": "ZFP36L2",
  "gene_name": "mRNA decay activator protein ZFP36L2",
  "gene": "UniProtKB:P47974"
}